{
  "gene_name": "M-phase phosphoprotein 6",
  "gene_symbol": "MPHOSPH6",
  "gene": "UniProtKB:Q99547",
  "term_label": "Unknown molecular function",
  "term_id": "UNKNOWN:0001"
}